{
  "gene_name": "Pre-B-cell leukemia transcription factor 1",
  "gene_symbol": "PBX1",
  "gene": "UniProtKB:P40424",
  "term_id": "GO:0001228",
  "term_label": "DNA-binding transcription activator activity, RNA polymerase II-specific"
}